regulation of inclusion body assembly [GO:0090083] (biological process) Sources: GOC:BHF, GOC:dph, GOC:tb Subtypes: negative regulation of inclusion body assembly [GO:0090084], positive regulation of inclusion body assembly [GO:0090261], regulation of Lewy body formation [GO:0140122], GO:1902996 Definition: Any process that modulates the rate, frequency, or extent of inclusion body assembly. Inclusion body assembly is the aggregation, arrangement and bonding together of a set of components to form an inclusion body. Relationships: is a type of GO:0044087; is a type of GO:0051128; regulates GO:0070841